{
  "term_id": "GO:0007186",
  "term_label": "G protein-coupled receptor signaling pathway",
  "gene_symbol": "OR8B12",
  "gene": "UniProtKB:Q8NGG6",
  "gene_name": "Olfactory receptor 8B12"
}